Leydig cell differentiation [GO:0033327] (biological process) References: PMID:12050120 Sources: GOC:ln Relationships: is a type of developmental process involved in reproduction [GO:0003006]; is a type of cell differentiation [GO:0030154]; BFO_0000050 male gonad development [GO:0008584] Definition: The process in which a relatively unspecialized cell acquires specialized structural and/or functional features of a Leydig cell. A Leydig cell is a testosterone-secreting cell in the interstitial area, between the seminiferous tubules, in the testis.